epinephrine transport [GO:0048241] (biological process) Also known as: adrenaline transport Sources: GOC:jid Definition: The directed movement of epinephrine into, out of or within a cell, or between cells, by means of some agent such as a transporter or pore. Subtypes: epinephrine secretion [GO:0048242] Relationships: is_a GO:0015695; is a type of catecholamine transport [GO:0051937]